{
  "gene_name": "Coatomer subunit epsilon",
  "term_id": "GO:0006891",
  "term_label": "intra-Golgi vesicle-mediated transport",
  "gene": "UniProtKB:O14579",
  "gene_symbol": "COPE"
}